{
  "term_label": "mRNA binding",
  "gene": "UniProtKB:Q04637",
  "gene_name": "Eukaryotic translation initiation factor 4 gamma 1",
  "term_id": "GO:0003729",
  "gene_symbol": "EIF4G1"
}